{
  "gene_name": "Putative lipoyltransferase 2, mitochondrial",
  "term_label": "Unknown biological process",
  "gene": "UniProtKB:A6NK58",
  "term_id": "UNKNOWN:0002",
  "gene_symbol": "LIPT2"
}